{
  "term_label": "nucleus",
  "gene_symbol": "SPI1",
  "gene": "UniProtKB:P17947",
  "term_id": "GO:0005634",
  "gene_name": "Transcription factor PU.1"
}